{
  "term_id": "GO:0006508",
  "gene": "UniProtKB:Q9NQH7",
  "term_label": "proteolysis",
  "gene_symbol": "XPNPEP3",
  "gene_name": "Xaa-Pro aminopeptidase 3"
}